{
  "gene": "UniProtKB:Q96EZ8",
  "term_id": "GO:0045944",
  "gene_symbol": "MCRS1",
  "term_label": "positive regulation of transcription by RNA polymerase II",
  "gene_name": "Microspherule protein 1"
}